{
  "term_id": "GO:0009897",
  "gene_name": "Semaphorin-7A",
  "gene": "UniProtKB:O75326",
  "gene_symbol": "SEMA7A",
  "term_label": "external side of plasma membrane"
}